regulation of lipid storage [GO:0010883] (biological process) Sources: GOC:BHF, GOC:dph, GOC:tb Subtypes: GO:0010884, regulation of cholesterol storage [GO:0010885], GO:0010888, regulation of triglyceride storage [GO:0010889] Also known as: regulation of lipid sequestration Relationships: is a type of regulation of cellular process [GO:0050794]; regulates lipid storage [GO:0019915] Definition: Any process that modulates the rate, frequency or extent of lipid storage. Lipid storage is the accumulation and maintenance in cells or tissues of lipids, compounds soluble in organic solvents but insoluble or sparingly soluble in aqueous solvents. Lipid reserves can be accumulated during early developmental stages for mobilization and utilization at later stages of development.